{
  "gene": "UniProtKB:A6NG13",
  "gene_symbol": "MGAT4D",
  "term_label": "endoplasmic reticulum",
  "gene_name": "Alpha-1,3-mannosyl-glycoprotein 4-beta-N-acetylglucosaminyltransferase-like protein MGAT4D",
  "term_id": "GO:0005783"
}